{
  "gene_name": "SLAM family member 6",
  "gene": "UniProtKB:Q96DU3",
  "term_id": "GO:0009897",
  "gene_symbol": "SLAMF6",
  "term_label": "external side of plasma membrane"
}